{
  "gene_symbol": "C5orf34",
  "term_id": "UNKNOWN:0003",
  "term_label": "Unknown cellular component",
  "gene_name": "Uncharacterized protein C5orf34",
  "gene": "UniProtKB:Q96MH7"
}